{
  "gene_symbol": "CUEDC2",
  "term_id": "UNKNOWN:0003",
  "gene": "UniProtKB:Q9H467",
  "term_label": "Unknown cellular component",
  "gene_name": "CUE domain-containing protein 2"
}